{
  "gene_name": "Beta-parvin",
  "gene_symbol": "PARVB",
  "gene": "UniProtKB:Q9HBI1",
  "term_id": "GO:0030032",
  "term_label": "lamellipodium assembly"
}